{
  "gene_name": "Uncharacterized protein C1orf105",
  "gene_symbol": "C1orf105",
  "term_label": "Unknown molecular function",
  "term_id": "UNKNOWN:0001",
  "gene": "UniProtKB:O95561"
}